nucleoside binding [GO:0001882] (molecular function) Relationships: is a type of GO:0097367; is a type of heterocyclic compound binding [GO:1901363] Sources: GOC:hjd Definition: Binding to a nucleoside, a compound consisting of a purine or pyrimidine nitrogenous base linked either to ribose or deoxyribose. Subtypes: purine nucleoside binding [GO:0001883], pyrimidine nucleoside binding [GO:0001884], deoxyribonucleoside binding [GO:0032546], ribonucleoside binding [GO:0032549]